{
  "gene_symbol": "OR10A2",
  "gene_name": "Olfactory receptor 10A2",
  "term_label": "detection of chemical stimulus involved in sensory perception of smell",
  "term_id": "GO:0050911",
  "gene": "UniProtKB:Q9H208"
}